{
  "term_id": "UNKNOWN:0003",
  "gene_symbol": "EIF4A1",
  "gene_name": "Eukaryotic initiation factor 4A-I",
  "term_label": "Unknown cellular component",
  "gene": "UniProtKB:P60842"
}